{
  "gene_name": "Eosinophil cationic protein",
  "term_id": "GO:0002227",
  "gene_symbol": "RNASE3",
  "gene": "UniProtKB:P12724",
  "term_label": "innate immune response in mucosa"
}